adenine/adenine mispair binding [GO:0035484] (molecular function) Definition: Binding to a double-stranded DNA region containing an A/A mispair. Sources: GOC:bf, GOC:jh Also known as: A/A mispair binding Relationships: is a type of GO:0030983